negative regulation of growth of unicellular organism as a thread of attached cells [GO:0070785] (biological process) Subtypes: GO:2000218, negative regulation of pseudohyphal growth [GO:2000221] Relationships: is a type of regulation of growth of unicellular organism as a thread of attached cells [GO:0070784]; is a type of negative regulation of filamentous growth of a population of unicellular organisms [GO:1900429]; negatively regulates GO:0070783 Definition: Any process that decreases the frequency, rate or extent of the process in which cells remain attached after division and form thread-like filaments that may penetrate into a solid growth medium. Sources: GOC:mah